{
  "term_id": "UNKNOWN:0003",
  "gene_name": "Transmembrane and ubiquitin-like domain-containing protein 2",
  "term_label": "Unknown cellular component",
  "gene_symbol": "TMUB2",
  "gene": "UniProtKB:Q71RG4"
}